{
  "term_id": "GO:0043022",
  "gene": "UniProtKB:Q8NE35",
  "gene_name": "Cytoplasmic polyadenylation element-binding protein 3",
  "term_label": "ribosome binding",
  "gene_symbol": "CPEB3"
}